{
  "term_id": "GO:0045444",
  "gene_name": "Transmembrane protein 120B",
  "gene": "UniProtKB:A0PK00",
  "gene_symbol": "TMEM120B",
  "term_label": "fat cell differentiation"
}